{
  "term_label": "cytoplasm",
  "gene_symbol": "SEC14L6",
  "term_id": "GO:0005737",
  "gene_name": "Putative SEC14-like protein 6",
  "gene": "UniProtKB:B5MCN3"
}